threonine biosynthetic process [GO:0009088] (biological process) Sources: GOC:jl, ISBN:0198506732 Also known as: threonine anabolism, threonine biosynthesis, threonine formation, threonine synthesis Definition: The chemical reactions and pathways resulting in the formation of threonine (2-amino-3-hydroxybutyric acid), a polar, uncharged, essential amino acid found in peptide linkage in proteins. Relationships: is a type of threonine metabolic process [GO:0006566]; is a type of GO:0009067